K6-linked polyubiquitin modification-dependent protein binding [GO:0071796] (molecular function) Definition: Binding to a protein upon poly-ubiquitination formed by linkages between lysine residues at position 6 in the target protein. Relationships: is a type of polyubiquitin modification-dependent protein binding [GO:0031593] References: PMID:17525341, PMID:20351172 Sources: GOC:sp